alkaline phosphatase activity [GO:0004035] (molecular function) Definition: Catalysis of the reaction: a phosphate monoester + H2O = an alcohol + phosphate, with an alkaline pH optimum. Relationships: is_a phosphatase activity [GO:0016791] Also known as: glycerophosphatase activity, phosphomonoesterase activity, alkaline phenyl phosphatase activity, alkaline phosphohydrolase activity, alkaline phosphomonoesterase activity, orthophosphoric-monoester phosphohydrolase (alkaline optimum), phosphate-monoester phosphohydrolase (alkaline optimum) Sources: EC:3.1.3.1 Regulation: RO_0002213 by positive regulation of alkaline phosphatase activity [GO:0010694]